{
  "term_label": "regulation of transcription by RNA polymerase II",
  "term_id": "GO:0006357",
  "gene": "UniProtKB:Q7Z7K2",
  "gene_symbol": "ZNF467",
  "gene_name": "Zinc finger protein 467"
}